{
  "gene_symbol": "CXorf1",
  "term_label": "Unknown cellular component",
  "gene_name": "Putative transmembrane protein CXorf1",
  "gene": "UniProtKB:O96002",
  "term_id": "UNKNOWN:0003"
}